{
  "gene_symbol": "MAN1B1",
  "gene_name": "Endoplasmic reticulum mannosyl-oligosaccharide 1,2-alpha-mannosidase",
  "gene": "UniProtKB:Q9UKM7",
  "term_label": "endoplasmic reticulum",
  "term_id": "GO:0005783"
}